regulation of CD4-positive, alpha-beta T cell costimulation [GO:1900279] (biological process) Definition: Any process that modulates the frequency, rate or extent of CD4-positive, alpha-beta T cell costimulation. Sources: GOC:BHF, GOC:TermGenie, GOC:pr Also known as: regulation of CD4-positive, alpha beta T cell costimulation Relationships: is a type of regulation of CD4-positive, alpha-beta T cell activation [GO:2000514]; is a type of regulation of T cell costimulation [GO:2000523]; regulates GO:0035783 Subtypes: negative regulation of CD4-positive, alpha-beta T cell costimulation [GO:1900280], GO:1900281